{
  "gene_name": "Keratin, type II cytoskeletal 1",
  "gene_symbol": "KRT1",
  "gene": "UniProtKB:P04264",
  "term_label": "intermediate filament organization",
  "term_id": "GO:0045109"
}